{
  "gene_symbol": "VEGFB",
  "gene_name": "Vascular endothelial growth factor B",
  "term_label": "induction of positive chemotaxis",
  "gene": "UniProtKB:P49765",
  "term_id": "GO:0050930"
}